{
  "term_id": "GO:0007127",
  "gene_name": "Bcl-2-like protein 11",
  "gene": "UniProtKB:O43521",
  "gene_symbol": "BCL2L11",
  "term_label": "meiosis I"
}